{
  "term_label": "clathrin adaptor activity",
  "term_id": "GO:0035615",
  "gene_symbol": "DAB2",
  "gene": "UniProtKB:P98082",
  "gene_name": "Disabled homolog 2"
}